{
  "term_label": "TSC1-TSC2 complex",
  "term_id": "GO:0033596",
  "gene": "UniProtKB:Q92574",
  "gene_name": "Hamartin",
  "gene_symbol": "TSC1"
}